interleukin-8 receptor binding [GO:0005153] (molecular function) Also known as: IL-8, interleukin-8 receptor ligand Definition: Binding to an interleukin-8 receptor. Sources: GOC:go_curators Relationships: is_a CXCR chemokine receptor binding [GO:0045236] Subtypes: CXCR1 chemokine receptor binding [GO:0045237], CXCR2 chemokine receptor binding [GO:0045238]